{
  "gene_name": "Protein TAMALIN",
  "gene": "UniProtKB:Q7Z6J2",
  "gene_symbol": "TAMALIN",
  "term_id": "GO:0005886",
  "term_label": "plasma membrane"
}